{
  "gene_name": "Serine protease HTRA2, mitochondrial",
  "term_id": "GO:0043065",
  "gene": "UniProtKB:O43464",
  "gene_symbol": "HTRA2",
  "term_label": "positive regulation of apoptotic process"
}